{
  "term_id": "GO:0043596",
  "term_label": "nuclear replication fork",
  "gene": "UniProtKB:O75717",
  "gene_symbol": "WDHD1",
  "gene_name": "WD repeat and HMG-box DNA-binding protein 1"
}